{
  "gene_symbol": "FGF14",
  "gene": "UniProtKB:Q92915",
  "term_id": "GO:0022008",
  "term_label": "neurogenesis",
  "gene_name": "Fibroblast growth factor 14"
}